{
  "gene": "UniProtKB:Q16594",
  "gene_name": "Transcription initiation factor TFIID subunit 9",
  "term_label": "transcription factor TFIID complex",
  "term_id": "GO:0005669",
  "gene_symbol": "TAF9"
}